{
  "gene_symbol": "IGKV2-40",
  "gene": "UniProtKB:A0A087WW87",
  "term_label": "Unknown molecular function",
  "term_id": "UNKNOWN:0001",
  "gene_name": "Immunoglobulin kappa variable 2-40"
}